oxidoreductase activity, acting on iron-sulfur proteins as donors, dinitrogen as acceptor [GO:0016732] (molecular function) Relationships: is a type of oxidoreductase activity, acting on iron-sulfur proteins as donors [GO:0016730] Subtypes: nitrogenase activity [GO:0016163] Sources: GOC:jl Definition: Catalysis of an oxidation-reduction (redox) reaction in which an iron-sulfur protein acts as a hydrogen or electron donor and reduces dinitrogen.